{
  "term_label": "Unknown molecular function",
  "gene_symbol": "C1QTNF9",
  "gene": "UniProtKB:P0C862",
  "term_id": "UNKNOWN:0001",
  "gene_name": "Complement C1q and tumor necrosis factor-related protein 9A"
}